formate dehydrogenase (quinone) activity [GO:0036397] (molecular function) Relationships: is_a oxidoreductase activity, acting on CH or CH2 groups, quinone or similar compound as acceptor [GO:0033695] Sources: GOC:bhm, RHEA:48592 Also known as: Fdh-N activity, formate dehydrogenase-N activity, formate:quinone oxidoreductase activity Definition: Catalysis of the reaction: formate + a quinone = CO2 + a quinol.